plastid-encoded plastid RNA polymerase complex A [GO:0000343] (cellular component) Also known as: PEP-A Relationships: is a type of GO:0000427 References: PMID:10946105 Definition: A plastid-encoded DNA-directed RNA polymerase complex that resembles eubacterial multisubunit RNA polymerases, with a core composed of alpha, beta, and beta-prime subunits. An additional subunit, a sigma factor, is required for promoter recognition. PEP-A is generated from the PEP-B form during chloroplast maturation to generate a complex composed of at least thirteen polypeptides that is not sensitive to the antibiotic rifampicin, like its precursor form the PEP-B complex.